lymphoid progenitor cell differentiation [GO:0002320] (BP) Subtypes: natural killer cell progenitor differentiation [GO:0002321], GO:0002328, pro-T cell differentiation [GO:0002572] Definition: The process in which a precursor cell type acquires the specialized features of a lymphoid progenitor cell. Lymphoid progenitor cells include progenitor cells for any of the lymphoid lineages. References: PMID:16551251, PMID:16551264 Sources: GOC:add Regulation: regulated by regulation of lymphoid progenitor cell differentiation [GO:1905456]; negatively regulated by GO:1905457; positively regulated by GO:1905458 Relationships: is a type of hematopoietic progenitor cell differentiation [GO:0002244]